detection of symbiotic bacterium [GO:0009604] (biological process) Definition: The series of events in which a stimulus from a symbiotic bacterium, a bacterium living in close physical association with another organism, is received and converted into a molecular signal. Also known as: detection of symbiotic bacteria, perception of symbiotic bacteria, perception of symbiotic bacterium Relationships: is a type of detection of symbiont [GO:0009602]; is a type of response to symbiotic bacterium [GO:0009609]; is a type of detection of bacterium [GO:0016045] Sources: GOC:hb, ISBN:0198506732